{
  "term_label": "Unknown biological process",
  "gene_name": "GLIPR1-like protein 1",
  "gene_symbol": "GLIPR1L1",
  "term_id": "UNKNOWN:0002",
  "gene": "UniProtKB:Q6UWM5"
}